{
  "term_label": "release of cytochrome c from mitochondria",
  "gene_name": "Bcl-2-related protein A1",
  "gene_symbol": "BCL2A1",
  "term_id": "GO:0001836",
  "gene": "UniProtKB:Q16548"
}